{
  "term_id": "UNKNOWN:0002",
  "gene_symbol": "CRYBG1",
  "gene_name": "Beta_gamma crystallin domain-containing protein 1",
  "gene": "UniProtKB:Q9Y4K1",
  "term_label": "Unknown biological process"
}